{
  "gene_symbol": "HRH3",
  "term_label": "dendrite",
  "term_id": "GO:0030425",
  "gene": "UniProtKB:Q9Y5N1",
  "gene_name": "Histamine H3 receptor"
}